{
  "gene_symbol": "DPYSL2",
  "gene_name": "Dihydropyrimidinase-related protein 2",
  "gene": "UniProtKB:Q16555",
  "term_label": "cytosol",
  "term_id": "GO:0005829"
}